{
  "term_id": "GO:0051019",
  "term_label": "mitogen-activated protein kinase binding",
  "gene_symbol": "PPM1D",
  "gene": "UniProtKB:O15297",
  "gene_name": "Protein phosphatase 1D"
}